{
  "gene": "UniProtKB:Q8NDI1",
  "term_id": "GO:0031267",
  "term_label": "small GTPase binding",
  "gene_name": "EH domain-binding protein 1",
  "gene_symbol": "EHBP1"
}